{
  "gene_name": "Probable ATP-dependent RNA helicase DDX17",
  "gene": "UniProtKB:Q92841",
  "term_label": "RNA helicase activity",
  "gene_symbol": "DDX17",
  "term_id": "GO:0003724"
}